{
  "term_label": "5'-flap endonuclease activity",
  "gene_symbol": "SLX1A",
  "gene_name": "Structure-specific endonuclease subunit SLX1",
  "gene": "UniProtKB:Q9BQ83",
  "term_id": "GO:0017108"
}